{
  "term_label": "nucleus",
  "gene": "UniProtKB:Q9Y5R5",
  "gene_symbol": "DMRT2",
  "term_id": "GO:0005634",
  "gene_name": "Doublesex- and mab-3-related transcription factor 2"
}